negative regulation of pentadecane biosynthetic process [GO:1900888] (biological process) Definition: Any process that stops, prevents or reduces the frequency, rate or extent of pentadecane biosynthetic process. Sources: GOC:TermGenie, GOC:mengo_curators Also known as: down regulation of pentadecane biosynthetic process, down-regulation of pentadecane biosynthetic process, downregulation of pentadecane biosynthetic process, inhibition of pentadecane biosynthesis, inhibition of pentadecane biosynthetic process, inhibition of pentadecane synthesis, down regulation of pentadecane anabolism, down regulation of pentadecane biosynthesis, down regulation of pentadecane formation, down regulation of pentadecane synthesis, down-regulation of pentadecane anabolism, down-regulation of pentadecane biosynthesis, down-regulation of pentadecane formation, down-regulation of pentadecane synthesis, downregulation of pentadecane anabolism, downregulation of pentadecane biosynthesis, downregulation of pentadecane formation, downregulation of pentadecane synthesis, inhibition of pentadecane anabolism, inhibition of pentadecane formation, negative regulation of pentadecane anabolism, negative regulation of pentadecane biosynthesis, negative regulation of pentadecane formation, negative regulation of pentadecane synthesis Relationships: is a type of GO:1900887; is a type of negative regulation of alkane biosynthetic process [GO:1901578]; negatively regulates pentadecane biosynthetic process [GO:1900634]